{
  "term_id": "GO:0016020",
  "gene_name": "Amphoterin-induced protein 2",
  "term_label": "membrane",
  "gene_symbol": "AMIGO2",
  "gene": "UniProtKB:Q86SJ2"
}